{
  "gene": "UniProtKB:Q07687",
  "gene_symbol": "DLX2",
  "term_id": "GO:0030154",
  "gene_name": "Homeobox protein DLX-2",
  "term_label": "cell differentiation"
}